nitrite transmembrane transporter activity [GO:0015113] (molecular function) Sources: GOC:ai Also known as: nitrite/nitrate porter activity Definition: Enables the transfer of nitrite (NO2-) ions from one side of a membrane to the other. Relationships: is a type of transmembrane transporter activity [GO:0022857]; is part of nitrite transport [GO:0015707] Subtypes: GO:0015514